{
  "term_label": "spherical high-density lipoprotein particle",
  "term_id": "GO:0034366",
  "gene_name": "Apolipoprotein C-II",
  "gene_symbol": "APOC2",
  "gene": "UniProtKB:P02655"
}